deNEDDylase activity [GO:0019784] (molecular function) Relationships: is a type of ubiquitin-like protein peptidase activity [GO:0019783] Definition: An isopeptidase activity that cleaves NEDD8 from a target protein to which it is conjugated. Also known as: NEDD8-specific protease activity References: PMID:25628956 Sources: GOC:mah Subtypes: GO:0140757, metal-dependent deNEDDylase activity [GO:0140758]